{
  "gene_symbol": "ITGAE",
  "gene": "UniProtKB:P38570",
  "term_id": "GO:0009986",
  "gene_name": "Integrin alpha-E",
  "term_label": "cell surface"
}